negative regulation of neutrophil extravasation [GO:2000390] (biological process) Sources: GOC:BHF, GOC:mah Definition: Any process that stops, prevents or reduces the frequency, rate or extent of neutrophil extravasation. Relationships: is a type of negative regulation of cellular extravasation [GO:0002692]; is a type of GO:1902623; is a type of regulation of neutrophil extravasation [GO:2000389]; negatively regulates GO:0072672